{
  "term_label": "positive regulation of apoptotic process",
  "gene_symbol": "STK17A",
  "term_id": "GO:0043065",
  "gene": "UniProtKB:Q9UEE5",
  "gene_name": "Serine_threonine-protein kinase 17A"
}